{
  "gene_symbol": "ZCCHC3",
  "gene": "UniProtKB:Q9NUD5",
  "gene_name": "Zinc finger CCHC domain-containing protein 3",
  "term_id": "GO:0009597",
  "term_label": "detection of virus"
}